{
  "gene_symbol": "TRPV1",
  "gene": "UniProtKB:Q8NER1",
  "gene_name": "Transient receptor potential cation channel subfamily V member 1",
  "term_id": "GO:0005262",
  "term_label": "calcium channel activity"
}